{
  "gene": "UniProtKB:Q9NP85",
  "gene_symbol": "NPHS2",
  "term_id": "UNKNOWN:0001",
  "term_label": "Unknown molecular function",
  "gene_name": "Podocin"
}